{
  "gene": "UniProtKB:Q9BRQ8",
  "gene_name": "Ferroptosis suppressor protein 1",
  "term_id": "GO:0050660",
  "gene_symbol": "AIFM2",
  "term_label": "flavin adenine dinucleotide binding"
}